{
  "gene_name": "Probable inactive 1-aminocyclopropane-1-carboxylate synthase-like protein 2",
  "term_label": "amino acid metabolic process",
  "term_id": "GO:0006520",
  "gene": "UniProtKB:Q4AC99",
  "gene_symbol": "ACCSL"
}